{
  "gene_name": "Alpha-actinin-4",
  "gene": "UniProtKB:O43707",
  "gene_symbol": "ACTN4",
  "term_label": "muscle cell development",
  "term_id": "GO:0055001"
}